{
  "gene": "UniProtKB:Q6NUJ5",
  "gene_name": "PWWP domain-containing protein 2B",
  "gene_symbol": "PWWP2B",
  "term_id": "GO:0005634",
  "term_label": "nucleus"
}